{
  "gene_symbol": "STEAP1B",
  "term_label": "Unknown molecular function",
  "gene": "UniProtKB:Q6NZ63",
  "term_id": "UNKNOWN:0001",
  "gene_name": "STEAP family member 1B"
}